{
  "term_id": "GO:0006886",
  "gene": "UniProtKB:P40617",
  "term_label": "intracellular protein transport",
  "gene_symbol": "ARL4A",
  "gene_name": "ADP-ribosylation factor-like protein 4A"
}